{
  "term_label": "neuron projection",
  "term_id": "GO:0043005",
  "gene": "UniProtKB:Q8IWU9",
  "gene_symbol": "TPH2",
  "gene_name": "Tryptophan 5-hydroxylase 2"
}